{
  "gene_name": "HAUS augmin-like complex subunit 7",
  "term_id": "GO:0070652",
  "gene_symbol": "HAUS7",
  "gene": "UniProtKB:Q99871",
  "term_label": "HAUS complex"
}